{
  "term_label": "Unknown biological process",
  "gene": "UniProtKB:A0PJE2",
  "term_id": "UNKNOWN:0002",
  "gene_symbol": "DHRS12",
  "gene_name": "Dehydrogenase_reductase SDR family member 12"
}